cellular response to oxygen radical [GO:0071450] (biological process) Subtypes: cellular response to superoxide [GO:0071451] Sources: GOC:mah Relationships: is a type of response to oxygen radical [GO:0000305]; is a type of cellular response to reactive oxygen species [GO:0034614] Definition: Any process that results in a change in state or activity of a cell (in terms of movement, secretion, enzyme production, gene expression, etc.) as a result of an oxygen radical stimulus. An oxygen radical is any oxygen species that carries a free electron; examples include hydroxyl radicals and the superoxide anion.